{
  "gene": "UniProtKB:Q8IYB0",
  "gene_name": "Putative uncharacterized protein MGC39545",
  "term_label": "Unknown molecular function",
  "term_id": "UNKNOWN:0001",
  "gene_symbol": "Q8IYB0"
}